{
  "term_label": "regulation of bone mineralization",
  "gene_symbol": "ECM1",
  "gene": "UniProtKB:Q16610",
  "term_id": "GO:0030500",
  "gene_name": "Extracellular matrix protein 1"
}